{
  "gene": "UniProtKB:P59074",
  "gene_symbol": "CHMP4BP1",
  "gene_name": "Putative charged multivesicular body protein 4B-like protein CHMP4BP1",
  "term_label": "Unknown molecular function",
  "term_id": "UNKNOWN:0001"
}